{
  "gene_symbol": "UNKL",
  "term_id": "UNKNOWN:0003",
  "term_label": "Unknown cellular component",
  "gene_name": "Putative E3 ubiquitin-protein ligase UNKL",
  "gene": "UniProtKB:Q9H9P5"
}